{
  "term_label": "ubiquitin-protein transferase activity",
  "gene_symbol": "RMND5A",
  "gene": "UniProtKB:Q9H871",
  "term_id": "GO:0004842",
  "gene_name": "E3 ubiquitin-protein transferase RMND5A"
}